negative regulation of chondrocyte differentiation [GO:0032331] (BP) Relationships: is a type of regulation of chondrocyte differentiation [GO:0032330]; is a type of negative regulation of cell differentiation [GO:0045596]; is a type of negative regulation of cartilage development [GO:0061037]; negatively regulates GO:0002062 Also known as: down regulation of chondrocyte differentiation, down-regulation of chondrocyte differentiation, downregulation of chondrocyte differentiation, inhibition of chondrocyte differentiation Subtypes: GO:0061182 Sources: GOC:mah Definition: Any process that stops, prevents, or reduces the frequency, rate or extent of chondrocyte differentiation.